{
  "gene_name": "DnaJ homolog subfamily C member 12",
  "gene_symbol": "DNAJC12",
  "gene": "UniProtKB:Q9UKB3",
  "term_label": "cytoplasm",
  "term_id": "GO:0005737"
}